{
  "term_label": "RNA polymerase II-specific DNA-binding transcription factor binding",
  "gene_symbol": "ZFPM2",
  "gene_name": "Zinc finger protein ZFPM2",
  "term_id": "GO:0061629",
  "gene": "UniProtKB:Q8WW38"
}